Hsp90 deacetylation [GO:0070846] (BP) Sources: GOC:BHF, GOC:mah Definition: The modification of an Hsp90 protein by removal of acetyl groups. Relationships: is a type of protein deacetylation [GO:0006476]